{
  "gene_name": "Meiosis-specific coiled-coil domain-containing protein MEIOC",
  "term_label": "male meiosis I",
  "gene": "UniProtKB:A2RUB1",
  "gene_symbol": "MEIOC",
  "term_id": "GO:0007141"
}